left lung morphogenesis [GO:0060460] (BP) Relationships: is a type of lung morphogenesis [GO:0060425]; is part of left lung development [GO:0060459] Definition: The process in which anatomical structures of the left lung are generated and organized. Sources: GOC:dph